{
  "term_label": "MLL3/4 complex",
  "gene": "UniProtKB:Q6ZW49",
  "gene_symbol": "PAXIP1",
  "gene_name": "PAX-interacting protein 1",
  "term_id": "GO:0044666"
}